{
  "gene_name": "Deoxynucleotidyltransferase terminal-interacting protein 1",
  "term_label": "DNA binding",
  "gene": "UniProtKB:Q9H147",
  "term_id": "GO:0003677",
  "gene_symbol": "DNTTIP1"
}